{
  "gene_name": "Phospholipid-transporting ATPase VA",
  "term_id": "GO:0045332",
  "gene_symbol": "ATP10A",
  "term_label": "phospholipid translocation",
  "gene": "UniProtKB:O60312"
}